{
  "gene": "UniProtKB:Q5T9C2",
  "gene_symbol": "EEIG1",
  "gene_name": "Early estrogen-induced gene 1 protein",
  "term_label": "Unknown molecular function",
  "term_id": "UNKNOWN:0001"
}